5-formyltetrahydrofolate cyclo-ligase activity [GO:0030272] (molecular function) Also known as: 5-formyltetrahydrofolate cyclodehydrase, 5,10-methenyltetrahydrofolate synthetase activity, 5-Formyltetrahydrofolate cyclodehydrase activity, 5-formyltetrahydrofolate cyclo-ligase (ADP-forming), formyltetrahydrofolic cyclodehydrase activity, methenyl-THF synthetase activity Relationships: is_a cyclo-ligase activity [GO:0016882] Definition: Catalysis of the reaction: 5-formyltetrahydrofolate + ATP = 5,10-methenyltetrahydrofolate + ADP + H+ + phosphate. Sources: EC:6.3.3.2, RHEA:10488